{
  "gene_symbol": "IFT56",
  "term_label": "intraciliary anterograde transport",
  "gene": "UniProtKB:A0AVF1",
  "term_id": "GO:0035720",
  "gene_name": "Intraflagellar transport protein 56"
}